{
  "term_label": "epithelial cilium movement involved in extracellular fluid movement",
  "gene_symbol": "CCDC103",
  "term_id": "GO:0003351",
  "gene": "UniProtKB:Q8IW40",
  "gene_name": "Coiled-coil domain-containing protein 103"
}